{
  "gene": "UniProtKB:P23582",
  "term_id": "GO:0006182",
  "gene_symbol": "NPPC",
  "term_label": "cGMP biosynthetic process",
  "gene_name": "C-type natriuretic peptide"
}